basement membrane assembly [GO:0070831] (biological process) Note: Note that this term has no relationship to 'membrane assembly ; GO:0071709' because the basement membrane is not a lipid bilayer. Subtypes: basement membrane assembly involved in embryonic body morphogenesis [GO:2001197] Relationships: is a type of basement membrane organization [GO:0071711]; is a type of extracellular matrix assembly [GO:0085029] Definition: The aggregation, arrangement and bonding together of a set of components to form a basement membrane, a part of the extracellular region that consists of a thin layer of dense material found in various animal tissues interposed between the cells and the adjacent connective tissue. Sources: GOC:mah